{
  "term_label": "protein polyubiquitination",
  "term_id": "GO:0000209",
  "gene_name": "E3 ubiquitin-protein ligase Topors",
  "gene_symbol": "TOPORS",
  "gene": "UniProtKB:Q9NS56"
}